{
  "gene": "UniProtKB:Q969E8",
  "term_label": "Unknown molecular function",
  "gene_name": "Pre-rRNA-processing protein TSR2 homolog",
  "gene_symbol": "TSR2",
  "term_id": "UNKNOWN:0001"
}